negative regulation of vitamin D biosynthetic process [GO:0010957] (biological process) Relationships: is a type of GO:0010894; is a type of negative regulation of vitamin metabolic process [GO:0046137]; is a type of regulation of vitamin D biosynthetic process [GO:0060556]; negatively regulates vitamin D biosynthetic process [GO:0042368] Sources: GOC:BHF, GOC:dph, GOC:tb Definition: Any process that decreases the rate, frequency or extent of a vitamin D biosynthetic process. Vitamin D biosynthesis is the chemical reactions and pathways resulting in the formation of vitamin D, any of a group of related, fat-soluble compounds that are derived from delta-5,7 steroids and play a central role in calcium metabolism. Specific forms of vitamin D include calciferol (ergocalciferol; vitamin D2) and cholecalciferol (calciol; vitamin D3).